negative regulation of FACT complex assembly [GO:1905645] (BP) Definition: Any process that stops, prevents or reduces the frequency, rate or extent of FACT complex assembly. Also known as: down regulation of FACT complex assembly, down regulation of FACT complex formation, down regulation of Facilitates chromatin transcription complex assembly, down regulation of Facilitates chromatin transcription complex formation, down-regulation of FACT complex assembly, down-regulation of FACT complex formation, down-regulation of Facilitates chromatin transcription complex assembly, down-regulation of Facilitates chromatin transcription complex formation, downregulation of FACT complex assembly, downregulation of FACT complex formation, downregulation of Facilitates chromatin transcription complex assembly, downregulation of Facilitates chromatin transcription complex formation, negative regulation of FACT complex formation, negative regulation of Facilitates chromatin transcription complex assembly, negative regulation of Facilitates chromatin transcription complex formation, inhibition of FACT complex assembly, inhibition of FACT complex formation, inhibition of Facilitates chromatin transcription complex assembly, inhibition of Facilitates chromatin transcription complex formation References: PMID:20889714 Sources: GOC:TermGenie, GO_REF:0000058 Relationships: is_a negative regulation of protein-containing complex assembly [GO:0031333]; is a type of GO:1905644; negatively regulates GO:1905635